{
  "term_id": "GO:0007186",
  "gene_symbol": "OPN1MW",
  "gene": "UniProtKB:P04001",
  "term_label": "G protein-coupled receptor signaling pathway",
  "gene_name": "Medium-wave-sensitive opsin 1"
}